D-arabinose 1-dehydrogenase (NAD+) activity [GO:0047816] (molecular function) Definition: Catalysis of the reaction: D-arabinose + NAD+ = D-arabinono-1,4-lactone + NADH. Sources: RHEA:20457 Also known as: D-arabinose:NAD+ 1-oxidoreductase activity, NAD-pentose-dehydrogenase activity, arabinose(fucose)dehydrogenase activity Relationships: is a type of D-arabinose 1-dehydrogenase [NAD(P)+] activity [GO:0045290]